norepinephrine-epinephrine catabolic process in blood stream [GO:0001995] (biological process) Definition: The chemical reactions and pathways resulting in the breakdown of norepinephrine or epinephrine in the bloodstream. Sources: GOC:hjd Also known as: noradrenaline-adrenalin catabolic process in blood stream Relationships: is a type of epinephrine catabolic process [GO:0042419]; is part of regulation of systemic arterial blood pressure by norepinephrine-epinephrine [GO:0001993]